{
  "gene": "UniProtKB:C0HM01",
  "gene_symbol": "SEPTIN14P20",
  "term_label": "Unknown cellular component",
  "term_id": "UNKNOWN:0003",
  "gene_name": "Putative RNA-binding regulatory peptide"
}